omega-6 fatty acid desaturase activity [GO:0045485] (molecular function) Relationships: is a type of oxidoreductase activity, acting on paired donors, with incorporation or reduction of molecular oxygen [GO:0016705] Definition: Catalysis of the introduction of an omega-6 double bond into the fatty acid hydrocarbon chain. References: PMID:7846158